GTP cyclohydrolase activity [GO:0003933] (molecular function) Definition: Catalysis of the hydrolysis of the imidazole ring of GTP, releasing formate. Two C-N bonds are hydrolyzed and the pentase unit is isomerized. Sources: GOC:curators Relationships: is_a cyclohydrolase activity [GO:0019238] Subtypes: GTP cyclohydrolase I activity [GO:0003934], GTP cyclohydrolase II activity [GO:0003935], GTP cyclohydrolase IIa activity [GO:0043740], GTP cyclohydrolase IV activity [GO:0044682]